{
  "term_id": "GO:0005762",
  "gene_name": "Large ribosomal subunit protein mL44",
  "gene": "UniProtKB:Q9H9J2",
  "gene_symbol": "MRPL44",
  "term_label": "mitochondrial large ribosomal subunit"
}